regulation of insulin secretion [GO:0050796] (biological process) Relationships: is_a regulation of protein secretion [GO:0050708]; is a type of regulation of peptide hormone secretion [GO:0090276]; regulates insulin secretion [GO:0030073] Sources: GOC:ai Definition: Any process that modulates the frequency, rate or extent of the regulated release of insulin. Subtypes: positive regulation of insulin secretion [GO:0032024], negative regulation of insulin secretion [GO:0046676], GO:0061178